{
  "gene_name": "Melanoma-associated antigen 1",
  "term_label": "nucleus",
  "gene": "UniProtKB:P43355",
  "term_id": "GO:0005634",
  "gene_symbol": "MAGEA1"
}